protein-cysteine S-palmitoyltransferase activity [GO:0019706] (MF) Also known as: protein-cysteine S-palmitoleyltransferase activity Relationships: is a type of palmitoyltransferase activity [GO:0016409]; is a type of GO:0019707 Sources: GOC:ai, GOC:pr, RHEA:36683 Definition: Catalysis of the transfer of a palmitoyl (systematic name, hexadecanoyl) group to a sulfur atom on the cysteine of a protein molecule, in the reaction hexadecanoyl-CoA + L-cysteinyl-[protein] = CoA + S-hexadecanoyl-L-cysteinyl-[protein]. Subtypes: GO:0043849